{
  "gene_symbol": "LINC01619",
  "gene": "UniProtKB:G3V211",
  "term_id": "UNKNOWN:0001",
  "term_label": "Unknown molecular function",
  "gene_name": "Uncharacterized protein encoded by LINC01619"
}